negative regulation of synapse pruning [GO:1905807] (BP) Definition: Any process that stops, prevents or reduces the frequency, rate or extent of synapse pruning. Also known as: regulation of synapse clearance, regulation of synapse disassembly, regulation of synapse elimination, regulation of synapse removal, down regulation of synapse disassembly, down-regulation of synapse disassembly, downregulation of synapse disassembly, inhibition of synapse disassembly References: PMID:27779093 Sources: GOC:TermGenie, GO_REF:0000058 Subtypes: negative regulation of excitatory synapse pruning [GO:1905811] Relationships: is a type of GO:1905806; is a type of negative regulation of synapse organization [GO:1905809]; negatively regulates synapse pruning [GO:0098883]